nicotine metabolic process [GO:0018933] (BP) Definition: The chemical reactions and pathways involving nicotine, (S)(-)-3-(1-methyl-2-pyrrolidinyl)pyridine. Also known as: nicotine metabolism Relationships: is a type of metabolic process [GO:0008152] Subtypes: GO:0019608, nicotine biosynthetic process [GO:0042179] Sources: GOC:sm, ISBN:0198547684